{
  "gene_name": "Immunoglobulin heavy variable 4-39",
  "term_label": "immunoglobulin mediated immune response",
  "term_id": "GO:0016064",
  "gene_symbol": "IGHV4-39",
  "gene": "UniProtKB:P01824"
}